{
  "gene_symbol": "TRPC7",
  "term_label": "regulation of cytosolic calcium ion concentration",
  "term_id": "GO:0051480",
  "gene": "UniProtKB:Q9HCX4",
  "gene_name": "Short transient receptor potential channel 7"
}